columnar/cuboidal epithelial cell differentiation [GO:0002065] (BP) Relationships: is a type of epithelial cell differentiation [GO:0030855] Definition: The process in which a relatively unspecialized cell acquires specialized features of a columnar/cuboidal epithelial cell. A columnar/cuboidal epithelial cell is a cell usually found in a two dimensional sheet with a free surface. Columnar/cuboidal epithelial cells take on the shape of a column or cube. Subtypes: glandular epithelial cell differentiation [GO:0002067], ameloblast differentiation [GO:0036305], neuroepithelial cell differentiation [GO:0060563], GO:0060575, multi-ciliated epithelial cell differentiation [GO:1903251] Sources: GOC:dph